stress fiber [GO:0001725] (cellular component) References: PMID:16651381 Definition: A contractile actin filament bundle that consists of short actin filaments with alternating polarity, cross-linked by alpha-actinin and possibly other actin bundling proteins, and with myosin present in a periodic distribution along the fiber. Also known as: stress fibre, actin cable Relationships: is a type of actomyosin [GO:0042641]; is a type of contractile actin filament bundle [GO:0097517]